{
  "term_label": "pyruvate import into mitochondria",
  "term_id": "GO:0006850",
  "gene": "UniProtKB:P0DKB6",
  "gene_name": "Mitochondrial pyruvate carrier 1-like protein",
  "gene_symbol": "MPC1L"
}